{
  "term_label": "Unknown biological process",
  "gene_symbol": "AMBP",
  "term_id": "UNKNOWN:0002",
  "gene": "UniProtKB:P02760",
  "gene_name": "Protein AMBP"
}